{
  "gene_name": "NADH dehydrogenase [ubiquinone] 1 alpha subcomplex subunit 10, mitochondrial",
  "term_label": "NADH dehydrogenase (ubiquinone) activity",
  "gene_symbol": "NDUFA10",
  "term_id": "GO:0008137",
  "gene": "UniProtKB:O95299"
}